negative T cell selection [GO:0043383] (biological process) Definition: The process of elimination of immature T cells which react strongly with self-antigens. Subtypes: GO:0045060, negative extrathymic T cell selection [GO:0045068] References: PMID:12414722 Sources: ISBN:0781735149 Also known as: negative T lymphocyte selection, negative T-cell selection, negative T-lymphocyte selection Relationships: is_a T cell selection [GO:0045058]